{
  "term_id": "GO:0000978",
  "gene_symbol": "ZNF710",
  "term_label": "RNA polymerase II cis-regulatory region sequence-specific DNA binding",
  "gene": "UniProtKB:Q8N1W2",
  "gene_name": "Zinc finger protein 710"
}